exhausted T cell differentiation [GO:0160083] (biological process) Definition: The process in which an activated T cell acquires specialized features of an exhausted T cell. Also known as: T cell exhaustion, T cell dysfuction References: PMID:21739672, PMID:31570879 Relationships: is a type of T cell differentiation [GO:0030217]